{
  "gene": "UniProtKB:Q6P995",
  "term_label": "Unknown cellular component",
  "gene_name": "Protein FAM171B",
  "gene_symbol": "FAM171B",
  "term_id": "UNKNOWN:0003"
}